{
  "term_label": "endoplasmic reticulum membrane",
  "gene_name": "DnaJ homolog subfamily B member 14",
  "gene_symbol": "DNAJB14",
  "gene": "UniProtKB:Q8TBM8",
  "term_id": "GO:0005789"
}